{
  "term_label": "Unknown molecular function",
  "gene": "UniProtKB:Q9H7C4",
  "gene_symbol": "SYNC",
  "term_id": "UNKNOWN:0001",
  "gene_name": "Syncoilin"
}